regulation of L-methionine import across plasma membrane [GO:1905624] (biological process) Subtypes: negative regulation of L-methionine import across plasma membrane [GO:1905625], GO:1905626 Relationships: is a type of regulation of amino acid import across plasma membrane [GO:0010958]; is a type of regulation of organic acid transport [GO:0032890]; regulates L-methionine import across plasma membrane [GO:1905544] Definition: Any process that modulates the frequency, rate or extent of L-methionine import across plasma membrane. References: PMID:17556368 Sources: GOC:TermGenie, GO_REF:0000058